oxidoreductase activity, acting on iron-sulfur proteins as donors [GO:0016730] (molecular function) Sources: GOC:ai Subtypes: oxidoreductase activity, acting on iron-sulfur proteins as donors, NAD or NADP as acceptor [GO:0016731], oxidoreductase activity, acting on iron-sulfur proteins as donors, dinitrogen as acceptor [GO:0016732], pheophorbide a oxygenase activity [GO:0032441] Definition: Catalysis of an oxidation-reduction (redox) reaction in which an iron-sulfur protein acts as a hydrogen or electron donor and reduces a hydrogen or electron acceptor. Relationships: is a type of GO:0016491 Also known as: oxidoreductase activity, acting on iron-sulphur proteins as donors